trihydroxytoluene dioxygenase activity [GO:0018616] (molecular function) References: PMID:1254564 Sources: UM-BBD_reactionID:r0093 Definition: Catalysis of the reaction: 2,3,5-trihydroxytoluene + O2 = 2,4,6-trioxoheptanoate. Relationships: is_a oxidoreductase activity, acting on paired donors, with incorporation or reduction of molecular oxygen, NAD(P)H as one donor, and incorporation of two atoms of oxygen into one donor [GO:0016708]